{
  "gene_name": "Flotillin-2",
  "gene": "UniProtKB:Q14254",
  "term_id": "GO:0016600",
  "term_label": "flotillin complex",
  "gene_symbol": "FLOT2"
}